{
  "gene_name": "MAP kinase-activated protein kinase 5",
  "term_id": "GO:0007265",
  "gene": "UniProtKB:Q8IW41",
  "gene_symbol": "MAPKAPK5",
  "term_label": "Ras protein signal transduction"
}